{
  "gene_name": "Rho-related GTP-binding protein RhoB",
  "gene": "UniProtKB:P62745",
  "term_label": "signal transduction",
  "term_id": "GO:0007165",
  "gene_symbol": "RHOB"
}